alcohol biosynthetic process [GO:0046165] (biological process) Definition: The chemical reactions and pathways resulting in the formation of alcohols, any of a class of compounds containing one or more hydroxyl groups attached to a saturated carbon atom. Sources: GOC:ai Also known as: alcohol anabolism, alcohol biosynthesis, alcohol formation, alcohol synthesis Relationships: is a type of GO:0006066; is a type of small molecule biosynthetic process [GO:0044283] Subtypes: amino acid catabolic process to alcohol via Ehrlich pathway [GO:0000947], octopamine biosynthetic process [GO:0006589], prenol biosynthetic process [GO:0016091], GO:0016094, cyclopentanol biosynthetic process [GO:0033021], GO:0034309, polyol biosynthetic process [GO:0046173], patulin biosynthetic process [GO:0140723], GO:1900769, monensin A biosynthetic process [GO:1901730], GO:1902645, secondary alcohol biosynthetic process [GO:1902653], fatty alcohol biosynthetic process [GO:1903175] Regulation: regulated by regulation of alcohol biosynthetic process [GO:1902930]; RO_0002212 by GO:1902931; positively regulated by GO:1902932